{
  "gene": "UniProtKB:Q8NGF1",
  "term_id": "GO:0004984",
  "gene_name": "Olfactory receptor 52R1",
  "term_label": "olfactory receptor activity",
  "gene_symbol": "OR52R1"
}